{
  "gene_name": "ARF GTPase-activating protein GIT2",
  "term_id": "GO:0032012",
  "gene": "UniProtKB:Q14161",
  "gene_symbol": "GIT2",
  "term_label": "regulation of ARF protein signal transduction"
}